{
  "gene": "UniProtKB:Q6PHR2",
  "term_label": "reticulophagy",
  "gene_symbol": "ULK3",
  "gene_name": "Serine_threonine-protein kinase ULK3",
  "term_id": "GO:0061709"
}